{
  "gene_symbol": "FGFR2",
  "gene_name": "Fibroblast growth factor receptor 2",
  "gene": "UniProtKB:P21802",
  "term_label": "plasma membrane",
  "term_id": "GO:0005886"
}